{
  "gene_symbol": "ZDHHC16",
  "term_label": "DNA damage response",
  "term_id": "GO:0006974",
  "gene_name": "Palmitoyltransferase ZDHHC16",
  "gene": "UniProtKB:Q969W1"
}